{
  "gene_name": "Protein mago nashi homolog",
  "term_label": "exon-exon junction complex",
  "term_id": "GO:0035145",
  "gene": "UniProtKB:P61326",
  "gene_symbol": "MAGOH"
}